{
  "gene": "UniProtKB:P43405",
  "gene_symbol": "SYK",
  "gene_name": "Tyrosine-protein kinase SYK",
  "term_label": "B cell receptor signaling pathway",
  "term_id": "GO:0050853"
}